negative regulation of calcium-dependent cell-cell adhesion [GO:0046588] (BP) Definition: Any process that stops, prevents, or reduces the frequency, rate or extent of calcium-dependent cell-cell adhesion. Sources: GOC:ai Also known as: down regulation of calcium-dependent cell-cell adhesion, down-regulation of calcium-dependent cell-cell adhesion, downregulation of calcium-dependent cell-cell adhesion, inhibition of calcium-dependent cell-cell adhesion Relationships: is a type of negative regulation of cell-cell adhesion [GO:0022408]; is a type of regulation of calcium-dependent cell-cell adhesion [GO:0046586]; negatively regulates calcium-dependent cell-cell adhesion [GO:0016339]